CAA codon-amino acid adaptor activity [GO:0033427] (molecular function) Sources: GOC:mah Note: Note that in the standard genetic code, CAA codes for glutamine. Also known as: glutamine tRNA Relationships: is a type of triplet codon-amino acid adaptor activity [GO:0030533] Definition: A triplet codon-amino acid adaptor activity that recognizes a CAA codon.